{
  "gene_symbol": "CNTNAP4",
  "gene_name": "Contactin-associated protein-like 4",
  "term_id": "GO:0045202",
  "term_label": "synapse",
  "gene": "UniProtKB:Q9C0A0"
}